{
  "term_label": "positive regulation of cell-substrate adhesion",
  "gene": "UniProtKB:Q76M96",
  "gene_name": "Coiled-coil domain-containing protein 80",
  "gene_symbol": "CCDC80",
  "term_id": "GO:0010811"
}